{
  "gene_symbol": "NDUFS8",
  "gene": "UniProtKB:O00217",
  "term_id": "GO:0032981",
  "term_label": "mitochondrial respiratory chain complex I assembly",
  "gene_name": "NADH dehydrogenase [ubiquinone] iron-sulfur protein 8, mitochondrial"
}